{
  "gene": "UniProtKB:O00267",
  "term_label": "DSIF complex",
  "gene_symbol": "SUPT5H",
  "gene_name": "Transcription elongation factor SPT5",
  "term_id": "GO:0032044"
}